{
  "term_label": "Unknown molecular function",
  "gene_name": "Archaemetzincin-2",
  "gene_symbol": "AMZ2",
  "gene": "UniProtKB:Q86W34",
  "term_id": "UNKNOWN:0001"
}